valine-3-methyl-2-oxovalerate transaminase activity [GO:0047301] (molecular function) Also known as: valine-3-methyl-2-oxovalerate aminotransferase activity, L-valine:(S)-3-methyl-2-oxopentanoate aminotransferase activity, valine--3-methyl-2-oxovalerate aminotransferase activity, valine--isoleucine aminotransferase activity, valine--isoleucine transaminase activity, valine-2-keto-methylvalerate aminotransferase activity Sources: EC:2.6.1.32, RHEA:11468 Relationships: is a type of transaminase activity [GO:0008483] Definition: Catalysis of the reaction: (S)-3-methyl-2-oxopentanoate + L-valine = 3-methyl-2-oxobutanoate + L-isoleucine.